{
  "gene_name": "Kinesin-like protein KIF6",
  "term_id": "GO:0007018",
  "term_label": "microtubule-based movement",
  "gene_symbol": "KIF6",
  "gene": "UniProtKB:Q6ZMV9"
}